{
  "term_id": "GO:0006298",
  "gene": "UniProtKB:P54278",
  "gene_symbol": "PMS2",
  "gene_name": "Mismatch repair endonuclease PMS2",
  "term_label": "mismatch repair"
}